{
  "term_label": "cellular response to interferon-beta",
  "gene_name": "Myeloid cell nuclear differentiation antigen",
  "term_id": "GO:0035458",
  "gene": "UniProtKB:P41218",
  "gene_symbol": "MNDA"
}